isoprenoid metabolic process [GO:0006720] (biological process) Regulation: regulated by regulation of isoprenoid metabolic process [GO:0019747]; negatively regulated by negative regulation of isoprenoid metabolic process [GO:0045827]; positively regulated by positive regulation of isopentenyl diphosphate biosynthetic process, mevalonate pathway [GO:1900486] Sources: ISBN:0198547684 Definition: The chemical reactions and pathways involving isoprenoid compounds, isoprene (2-methylbuta-1,3-diene) or compounds containing or derived from linked isoprene (3-methyl-2-butenylene) residues. Relationships: is a type of GO:0006629 Also known as: isoprenoid metabolism, polyisoprenoid metabolic process, polyisoprenoid metabolism, polyterpene metabolic process, polyterpene metabolism Subtypes: terpenoid metabolic process [GO:0006721], isoprenoid biosynthetic process [GO:0008299], GO:0008300, polyprenol metabolic process [GO:0016093], terpene metabolic process [GO:0042214]